{
  "term_id": "GO:0005634",
  "gene_name": "Doublesex- and mab-3-related transcription factor C1",
  "term_label": "nucleus",
  "gene": "UniProtKB:Q5HYR2",
  "gene_symbol": "DMRTC1"
}